{
  "term_label": "Unknown cellular component",
  "term_id": "UNKNOWN:0003",
  "gene_symbol": "FAM240A",
  "gene": "UniProtKB:A0A1B0GVK7",
  "gene_name": "Protein FAM240A"
}